regulation of nuclear-transcribed mRNA catabolic process, nonsense-mediated decay [GO:2000622] (BP) Definition: Any process that modulates the frequency, rate or extent of nuclear-transcribed mRNA catabolic process, nonsense-mediated decay. Sources: GOC:obol Relationships: is a type of regulation of mRNA catabolic process [GO:0061013]; regulates nuclear-transcribed mRNA catabolic process, nonsense-mediated decay [GO:0000184] Also known as: regulation of mRNA breakdown, nonsense-mediated decay, regulation of mRNA catabolic process, nonsense-mediated, regulation of mRNA catabolism, nonsense-mediated, regulation of mRNA degradation, nonsense-mediated decay, regulation of nonsense-mediated mRNA decay, regulation of nuclear mRNA catabolic process, nonsense-mediated decay Subtypes: negative regulation of nuclear-transcribed mRNA catabolic process, nonsense-mediated decay [GO:2000623], positive regulation of nuclear-transcribed mRNA catabolic process, nonsense-mediated decay [GO:2000624]